{
  "gene": "UniProtKB:Q8IYX8",
  "term_id": "GO:0005813",
  "gene_name": "Centrosomal protein CEP57L1",
  "term_label": "centrosome",
  "gene_symbol": "CEP57L1"
}